ABC-type teichoic acid transporter activity [GO:0015438] (molecular function) References: PMID:7565096 Relationships: is a type of macromolecule transmembrane transporter activity [GO:0022884]; is a type of ABC-type transporter activity [GO:0140359]; is a type of carbohydrate derivative transmembrane transporter activity [GO:1901505]; is part of teichoic acid transport [GO:0015777] Also known as: teichoic acid transmembrane transporter activity, ABC-type teichoic-acid transporter, teichoic-acid ABC transporter, ATP-dependent teichoic acid transmembrane transporter activity, ATPase-coupled teichoic acid transmembrane transporter activity, teichoic-acid-transporting ATPase activity Definition: Enables the transfer of a solute or solutes from one side of a membrane to the other according to the reaction: ATP + H2O + teichoic acid(in) = ADP + phosphate + teichoic acid(out).